{
  "gene_symbol": "POLR2F",
  "term_label": "RNA polymerase III complex",
  "gene_name": "DNA-directed RNA polymerases I, II, and III subunit RPABC2",
  "gene": "UniProtKB:P61218",
  "term_id": "GO:0005666"
}